{
  "term_label": "dipeptidase activity",
  "gene_name": "Dipeptidase 1",
  "term_id": "GO:0016805",
  "gene": "UniProtKB:P16444",
  "gene_symbol": "DPEP1"
}